2-dehydro-3-deoxy-D-gluconate 5-dehydrogenase activity [GO:0047001] (molecular function) Definition: Catalysis of the reaction: NAD+ + 2-dehydro-3-deoxy-D-gluconate = NADH + (4S)-4,6-dihydroxy-2,5-dioxohexanoate. Also known as: 2-dehydro-3-deoxy-D-gluconate:NAD+ 5-oxidoreductase activity, 2-keto-3-deoxy-D-gluconate (3-deoxy-D-glycero-2,5-hexodiulosonic acid) dehydrogenase activity, 2-keto-3-deoxygluconate (nicotinamide adenine dinucleotide (phosphate)) dehydrogenase activity, 2-keto-3-deoxygluconate 5-dehydrogenase activity, 2-keto-3-deoxygluconate dehydrogenase activity Sources: EC:1.1.1.127, MetaCyc:1.1.1.127-RXN Relationships: is a type of oxidoreductase activity, acting on the CH-OH group of donors, NAD or NADP as acceptor [GO:0016616]